ATP-dependent protein-DNA unloader activity [GO:0140083] (molecular function) References: PMID:28552615 Relationships: is a type of ATP-dependent activity, acting on DNA [GO:0008094] Also known as: ATP-dependent protein-DNA unloading activity, protein-DNA unloading ATPase activity Definition: Facilitating the removal of a protein or protein complex from a DNA molecule driven by ATP hydrolysis. This can be achieved for example by introducing non-canonical DNA structures or generating torque to directly inhibit a protein-DNA binding interaction. Subtypes: ATP-dependent protein-DNA complex displacement activity [GO:0061995]